{
  "gene": "UniProtKB:Q96HQ0",
  "term_id": "GO:0006357",
  "term_label": "regulation of transcription by RNA polymerase II",
  "gene_symbol": "ZNF419",
  "gene_name": "Zinc finger protein 419"
}